oxoglutarate dehydrogenase (succinyl-transferring) activity [GO:0004591] (molecular function) Sources: RHEA:12188 Definition: Catalysis of the reaction: N(6)-[(R)-lipoyl]-L-lysyl-[dihydrolipoyllysine-residue succinyltransferase] + 2-oxoglutarate + H+ = N(6)-[(R)-S(8)-succinyldihydrolipoyl]-L-lysyl-[dihydrolipoyllysine-residue succinyltransferase] + CO2. Also known as: oxoglutarate dehydrogenase (lipoamide) activity, 2-ketoglutarate dehydrogenase activity, 2-oxoglutarate dehydrogenase activity, 2-oxoglutarate: lipoate oxidoreductase activity, 2-oxoglutarate:dihydrolipoyllysine-residue succinyltransferase-lipoyllysine 2-oxidoreductase (decarboxylating, acceptor-succinylating), 2-oxoglutarate:lipoamide 2-oxidoreductase (decarboxylating and acceptor-succinylating) activity, AKGDH activity, OGDC activity, alpha-ketoglutarate dehydrogenase activity, alpha-ketoglutaric acid dehydrogenase activity, alpha-ketoglutaric dehydrogenase activity, alpha-oxoglutarate dehydrogenase activity, ketoglutaric dehydrogenase activity, oxoglutarate decarboxylase activity, oxoglutarate dehydrogenase activity Relationships: is a type of oxidoreductase activity, acting on the aldehyde or oxo group of donors, disulfide as acceptor [GO:0016624]